regulation of cytoplasmic translational fidelity [GO:0140018] (biological process) Relationships: is a type of regulation of translational fidelity [GO:0006450]; is a type of GO:1900247 References: PMID:22768388 Definition: Any process that modulates the ability of the cytoplasmic translational apparatus to interpret the genetic code.